L-asparagine catabolic process via L-aspartate [GO:0033345] (biological process) Definition: The chemical reactions and pathways resulting in the breakdown of L-asparagine, via the intermediate L-aspartate. Relationships: is a type of GO:0006530 Sources: GOC:mah